{
  "gene": "UniProtKB:Q9H6D3",
  "term_label": "apoptotic process involved in development",
  "gene_name": "XK-related protein 8",
  "gene_symbol": "XKR8",
  "term_id": "GO:1902742"
}